2-amino-5-formylamino-6-(5-phosphoribosylamino)pyrimidin-4(3H)-one formate-lyase activity [GO:0043729] (molecular function) Definition: Catalysis of the reaction: 2-amino-5-formylamino-6-(5-phospho-D-ribosylamino)pyrimidin-4(3H)-one + H2O = 2,5-diamino-6-(1-D-ribosylamino)pyrimidin-4(3H)-one 5'-phosphate + formate + H+. Relationships: is_a GO:0016811 Sources: RHEA:27282